{
  "gene": "UniProtKB:Q8TE02",
  "term_label": "tRNA binding",
  "gene_name": "Elongator complex protein 5",
  "term_id": "GO:0000049",
  "gene_symbol": "ELP5"
}